ABC-type beta-glucan transporter activity [GO:0015441] (molecular function) Sources: RHEA:18453 Also known as: beta-glucan ABC transporter, ABC-type beta-glucan transporter, ATP-dependent beta-glucan transporter activity, ATPase-coupled beta-glucan transporter activity, beta-glucan-transporting ATPase activity Definition: Enables the transfer of a solute or solutes from one side of a membrane to the other according to the reaction: ATP + H2O + beta-glucan(in) = ADP + phosphate + beta-glucan(out). Relationships: is a type of beta-glucan transmembrane transporter activity [GO:0015160]; is a type of GO:0043211